{
  "term_label": "protein-RNA adaptor activity",
  "gene_symbol": "ELAVL4",
  "term_id": "GO:0140517",
  "gene": "UniProtKB:P26378",
  "gene_name": "ELAV-like protein 4"
}